regulation of stress granule assembly [GO:0062028] (biological process) References: PMID:20180778 Subtypes: positive regulation of stress granule assembly [GO:0062029], negative regulation of stress granule assembly [GO:0062030] Definition: Any process that modulates the rate, frequency or extent of stress granule assembly, the aggregation, arrangement and bonding together of proteins and RNA molecules to form a stress granule. Relationships: is a type of GO:1902115; RO_0002211 stress granule assembly [GO:0034063]